{
  "gene_name": "Migration and invasion enhancer 1",
  "term_id": "GO:0051491",
  "gene_symbol": "MIEN1",
  "term_label": "positive regulation of filopodium assembly",
  "gene": "UniProtKB:Q9BRT3"
}